tolerance induction in gut-associated lymphoid tissue [GO:0002394] (biological process) Definition: Tolerance induction taking place in the gut-associated lymphoid tissue (GALT). Sources: GOC:jal, ISBN:0781735149 Also known as: tolerance induction in GALT, oral tolerance Relationships: is a type of immune response in gut-associated lymphoid tissue [GO:0002387]; is a type of tolerance induction in mucosal-associated lymphoid tissue [GO:0002401] Subtypes: GO:0002389, tolerance induction in nasopharyngeal-associated lymphoid tissue [GO:0002400]